regulation of convergent extension involved in neural plate elongation [GO:1904130] (biological process) Relationships: is a type of regulation of convergent extension involved in gastrulation [GO:1904103]; regulates GO:0022007 Subtypes: negative regulation of convergent extension involved in neural plate elongation [GO:1904131], positive regulation of convergent extension involved in neural plate elongation [GO:1904132] Definition: Any process that modulates the frequency, rate or extent of convergent extension involved in neural plate elongation. References: PMID:24892953 Sources: GOC:TermGenie, GOC:dph, GO_REF:0000058